{
  "gene": "UniProtKB:Q9BRQ8",
  "term_id": "GO:0008637",
  "gene_symbol": "AIFM2",
  "term_label": "apoptotic mitochondrial changes",
  "gene_name": "Ferroptosis suppressor protein 1"
}